{
  "term_label": "cytosol",
  "gene_symbol": "GAPDH",
  "gene": "UniProtKB:P04406",
  "gene_name": "Glyceraldehyde-3-phosphate dehydrogenase",
  "term_id": "GO:0005829"
}